metanephric capsule morphogenesis [GO:0072265] (BP) Sources: GOC:mtg_kidney_jan10 Relationships: is a type of GO:0072128; is part of metanephric capsule development [GO:0072213] Definition: The process in which the anatomical structures of the metanephric capsule are generated and organized. The metanephric capsule is the tough fibrous layer surrounding the metanephros, covered in a thick layer of perinephric adipose tissue. It provides some protection from trauma and damage.